{
  "gene_name": "Putative uncharacterized protein C6orf52",
  "gene": "UniProtKB:Q5T4I8",
  "term_id": "UNKNOWN:0002",
  "gene_symbol": "C6orf52",
  "term_label": "Unknown biological process"
}